regulation of leukocyte tethering or rolling [GO:1903236] (biological process) Subtypes: negative regulation of leukocyte tethering or rolling [GO:1903237], positive regulation of leukocyte tethering or rolling [GO:1903238] Relationships: is a type of GO:0002691; is a type of GO:1904994; regulates GO:0050901 References: PMID:18308860 Sources: GOC:TermGenie, GOC:als, GO_REF:0000058 Definition: Any process that modulates the frequency, rate or extent of leukocyte tethering or rolling.